nuclear receptor-mediated bile acid signaling pathway [GO:0038185] (BP) Also known as: FXR signaling pathway, farnesoid X receptor signaling pathway, intracellular bile acid receptor signaling pathway, BAR signaling pathway, nuclear bile acid receptor signaling pathway Definition: A nuclear receptor-mediated signaling pathway initiated by a bile acid binding to an intracellular receptor of the nuclear receptor protein family, and ending with regulation of a downstream cellular process, e.g. transcription. Relationships: is a type of bile acid signaling pathway [GO:0038183]; is a type of GO:0141193; has part bile acid nuclear receptor activity [GO:0038186] References: PMID:10334992, PMID:36409000